ceramide-1-phosphate phosphatase activity [GO:0106235] (molecular function) References: PMID:10359651 Sources: GOC:lb Relationships: is a type of lipid phosphatase activity [GO:0042577] Definition: Catalysis of the reaction: ceramide-1-phosphate + H2O = ceramide+ phosphate.